{
  "term_id": "UNKNOWN:0002",
  "gene": "UniProtKB:Q86W74",
  "gene_symbol": "ANKRD46",
  "term_label": "Unknown biological process",
  "gene_name": "Ankyrin repeat domain-containing protein 46"
}